{
  "gene_symbol": "ABCG2",
  "term_id": "GO:0015562",
  "gene": "UniProtKB:Q9UNQ0",
  "gene_name": "Broad substrate specificity ATP-binding cassette transporter ABCG2",
  "term_label": "efflux transmembrane transporter activity"
}